{
  "gene_symbol": "PARD6B",
  "term_label": "cell cortex",
  "gene_name": "Partitioning defective 6 homolog beta",
  "gene": "UniProtKB:Q9BYG5",
  "term_id": "GO:0005938"
}